{
  "term_id": "GO:0009897",
  "gene": "UniProtKB:Q6ZS10",
  "gene_symbol": "CLEC17A",
  "term_label": "external side of plasma membrane",
  "gene_name": "C-type lectin domain family 17, member A"
}